L-lactate dehydrogenase (NAD+) activity [GO:0004459] (molecular function) Definition: Catalysis of the reaction: (S)-lactate + NAD+ = pyruvate + NADH + H+. Relationships: is a type of L-2-hydroxycarboxylate dehydrogenase (NAD+) activity [GO:0102443]; is a type of L-lactate dehydrogenase activity [GO:0140171] Regulation: negatively regulated by L-lactate dehydrogenase inhibitor activity [GO:0160193] Also known as: L-lactate dehydrogenase activity, L-lactic acid dehydrogenase activity, L-lactic dehydrogenase activity Sources: RHEA:23444